B-1a B cell differentiation [GO:0002337] (biological process) Note: Note that immunologists typically use the word 'development' to refer to cells of B or T cell lineages undergoing the process that GO describes as 'cell differentiation'. Sources: GOC:jal, ISBN:0781735149 Also known as: B-1a B lymphocyte differentiation, B-1a B-cell differentiation, B-1a B-lymphocyte differentiation, B-1a B cell development Relationships: is_a B-1 B cell differentiation [GO:0001923] Definition: The process in which B cells acquire the specialized features of B-1a B cells. B-1a B cells are B-1 cells that express CD5 and arise from fetal liver precursors.